m-cresol catabolic process [GO:0042213] (biological process) Definition: The chemical reactions and pathways resulting in the breakdown of m-cresol (3-hydroxytoluene), the meta-isoform of cresol. Sources: GOC:jl Also known as: 3-hydroxytoluene catabolic process, 3-hydroxytoluene catabolism, m-cresol breakdown, m-cresol catabolism, m-cresol degradation, meta-cresol catabolic process, meta-cresol catabolism Relationships: is a type of GO:0046199